{
  "gene_name": "Zinc finger protein 32",
  "term_id": "GO:0000978",
  "gene_symbol": "ZNF32",
  "term_label": "RNA polymerase II cis-regulatory region sequence-specific DNA binding",
  "gene": "UniProtKB:P17041"
}